{
  "term_id": "GO:0005576",
  "term_label": "extracellular region",
  "gene_name": "Extracellular tyrosine-protein kinase PKDCC",
  "gene_symbol": "PKDCC",
  "gene": "UniProtKB:Q504Y2"
}